Rhino-Deadlock-Cutoff Complex [GO:1990469] (cellular component) Note: An example of this is cuff in Drosophila melanogaster (Q9V629) in PMID:24906153. References: PMID:24906153 Sources: GOC:bhm Also known as: RDC complex, rhi-del-cuff complex Relationships: is a type of GO:0140513; is a type of PET complex [GO:1990923]; is part of germ cell nucleus [GO:0043073] Definition: Protein complex found in Drosophila consisting of the gene products of cuff, del and rhi. It regulates the licensing of transcription of dual-strand PIWI interacting RNA (piRNA) source loci by binding to dual-strand-cluster chromatin, probably via the H3K9me3-binding activity of Rhi. Rhi binding brings the putative termination cofactor Cuff in close proximity to the nascent piRNA precursor transcript which it appears to protect from degradation.